{
  "term_label": "extracellular matrix structural constituent conferring tensile strength",
  "gene_name": "Collagen alpha-1(IX) chain",
  "gene_symbol": "COL9A1",
  "term_id": "GO:0030020",
  "gene": "UniProtKB:P20849"
}